{
  "term_label": "cytoplasm",
  "gene_name": "Tumor necrosis factor alpha-induced protein 8-like protein 2",
  "term_id": "GO:0005737",
  "gene_symbol": "TNFAIP8L2",
  "gene": "UniProtKB:Q6P589"
}